{
  "gene": "UniProtKB:Q8NGS0",
  "term_id": "GO:0005886",
  "gene_name": "Olfactory receptor 1N1",
  "gene_symbol": "OR1N1",
  "term_label": "plasma membrane"
}